MHC class I peptide loading complex [GO:0042824] (cellular component) Note: Note that although this complex is located in the endoplasmic reticulum, there is some evidence that it may also be found in the Golgi. Definition: A large, multisubunit complex which consists of the MHC class I-beta 2 microglobulin dimer, the transporter associated with antigen presentation (TAP), tapasin (an MHC-encoded membrane protein), the chaperone calreticulin and the thiol oxidoreductase ERp57. Functions in the assembly of peptides with newly synthesized MHC class I molecules. Also known as: peptide-loading complex, PLC Relationships: is a type of membrane protein complex [GO:0098796]; is a type of endoplasmic reticulum protein-containing complex [GO:0140534]; is part of endoplasmic reticulum membrane [GO:0005789] References: PMID:10631934 Sources: GOC:jl